{
  "gene_symbol": "ACSM1",
  "term_label": "fatty acid ligase activity",
  "gene": "UniProtKB:Q08AH1",
  "term_id": "GO:0015645",
  "gene_name": "Acyl-coenzyme A synthetase ACSM1, mitochondrial"
}